{
  "gene": "UniProtKB:A8MZG2",
  "term_label": "Unknown biological process",
  "gene_symbol": "C16orf90",
  "term_id": "UNKNOWN:0002",
  "gene_name": "Uncharacterized protein C16orf90"
}